{
  "term_id": "UNKNOWN:0001",
  "term_label": "Unknown molecular function",
  "gene_symbol": "SAMM50",
  "gene_name": "Sorting and assembly machinery component 50 homolog",
  "gene": "UniProtKB:Q9Y512"
}